epithelial cell proliferation involved in prostatic bud elongation [GO:0060517] (biological process) Definition: The multiplication of epithelial cells, contributing to the expansion of the primary prostatic bud. References: PMID:18977204 Sources: GOC:dph Relationships: is a type of epithelial cell proliferation involved in prostate gland development [GO:0060767]; is part of primary prostatic bud elongation [GO:0060516]